pigment granule [GO:0048770] (cellular component) Relationships: is a type of cytoplasmic vesicle [GO:0031410] Sources: GOC:jid, GOC:mh Definition: A small, subcellular membrane-bounded vesicle containing pigment and/or pigment precursor molecules. Pigment granule biogenesis is poorly understood, as pigment granules are derived from multiple sources including the endoplasmic reticulum, coated vesicles, lysosomes, and endosomes. Subtypes: melanosome [GO:0042470], GO:0043698, leucosome [GO:0043699], GO:0043700, cyanosome [GO:0043701]